{
  "gene": "UniProtKB:Q6GV28",
  "term_id": "UNKNOWN:0003",
  "gene_symbol": "TMEM225",
  "gene_name": "Transmembrane protein 225",
  "term_label": "Unknown cellular component"
}